{
  "term_id": "UNKNOWN:0001",
  "gene_name": "Pyruvate dehydrogenase E1 component subunit alpha, somatic form, mitochondrial",
  "gene": "UniProtKB:P08559",
  "term_label": "Unknown molecular function",
  "gene_symbol": "PDHA1"
}